photosynthetic membrane [GO:0034357] (cellular component) Subtypes: thylakoid membrane [GO:0042651], plasma membrane-derived chromatophore membrane [GO:0042717] Definition: A membrane enriched in complexes formed of reaction centers, accessory pigments and electron carriers, in which photosynthetic reactions take place. Relationships: is a type of membrane [GO:0016020]; is part of thylakoid [GO:0009579] Sources: GOC:ds, GOC:mah